{
  "gene_name": "Olfactory receptor 52E6",
  "gene": "UniProtKB:Q96RD3",
  "gene_symbol": "OR52E6",
  "term_label": "olfactory receptor activity",
  "term_id": "GO:0004984"
}